{
  "term_label": "actin cytoskeleton organization",
  "gene_symbol": "PARVA",
  "gene_name": "Alpha-parvin",
  "gene": "UniProtKB:Q9NVD7",
  "term_id": "GO:0030036"
}